{
  "term_label": "response to cytokine",
  "term_id": "GO:0034097",
  "gene": "UniProtKB:P16109",
  "gene_symbol": "SELP",
  "gene_name": "P-selectin"
}